regulation of protein localization to cilium [GO:1903564] (biological process) References: PMID:22072986 Sources: GOC:TermGenie, GOC:cilia, GOC:krc, GO_REF:0000058 Relationships: is a type of regulation of protein localization [GO:0032880]; regulates protein localization to cilium [GO:0061512] Definition: Any process that modulates the frequency, rate or extent of protein localization to cilium. Subtypes: negative regulation of protein localization to cilium [GO:1903565], positive regulation of protein localization to cilium [GO:1903566], GO:1903567